L-arginine transmembrane export from vacuole [GO:1990818] (biological process) Relationships: is a type of organic cation transport [GO:0015695]; is a type of GO:0032974; is a type of L-alpha-amino acid transmembrane transport [GO:1902475] Definition: The directed movement of L-arginine out of the vacuole, across the vacuolar membrane. Subtypes: L-arginine transmembrane transport from lysosomal lumen to cytosol [GO:1904917] References: PMID:26083598